{
  "term_label": "microtubule binding",
  "gene": "UniProtKB:Q8N427",
  "gene_name": "Thioredoxin domain-containing protein 3",
  "term_id": "GO:0008017",
  "gene_symbol": "NME8"
}